{
  "gene_name": "Tudor domain-containing protein 1",
  "term_id": "UNKNOWN:0001",
  "term_label": "Unknown molecular function",
  "gene_symbol": "TDRD1",
  "gene": "UniProtKB:Q9BXT4"
}